{
  "gene_symbol": "LIG4",
  "gene": "UniProtKB:P49917",
  "gene_name": "DNA ligase 4",
  "term_id": "GO:0033152",
  "term_label": "immunoglobulin V(D)J recombination"
}